asymmetric synapse [GO:0032279] (CC) Definition: A type of synapse occurring between an axon and a dendritic spine or dendritic shaft. Asymmetric synapses, the most abundant synapse type in the central nervous system, involve axons that contain predominantly spherical vesicles and contain a thickened postsynaptic density. Most or all synapses of this type are excitatory. Sources: GOC:dgh, GOC:ef Subtypes: mossy fiber rosette [GO:0097471], asymmetric, glutamatergic, excitatory synapse [GO:0098985], spine synapse [GO:0106033] Relationships: is_a neuron to neuron synapse [GO:0098984]; has part postsynaptic density [GO:0014069] Also known as: Gray's type I synapse